{
  "gene": "UniProtKB:Q86TI4",
  "gene_name": "WD repeat-containing protein 86",
  "term_label": "Unknown biological process",
  "term_id": "UNKNOWN:0002",
  "gene_symbol": "WDR86"
}